{
  "gene": "UniProtKB:Q8TCU6",
  "gene_symbol": "PREX1",
  "term_id": "GO:0005085",
  "gene_name": "Phosphatidylinositol 3,4,5-trisphosphate-dependent Rac exchanger 1 protein",
  "term_label": "guanyl-nucleotide exchange factor activity"
}